sorocarp morphogenesis [GO:0031288] (biological process) Relationships: is a type of GO:0009653; is part of sorocarp development [GO:0030587] Also known as: fruiting body morphogenesis Definition: The process in which the sorocarp is generated and organized. An example of this process is found in Dictyostelium discoideum. References: PMID:4332228 Sources: GOC:kp, GOC:mtg_sensu